plasma membrane phospholipid scrambling [GO:0017121] (biological process) Subtypes: calcium activated phospholipid scrambling [GO:0061588], GO:0061592, phosphatidylserine exposure on apoptotic cell surface [GO:0070782], phosphatidylserine exposure on blood platelet [GO:0097045] References: PMID:20043909, PMID:20302864 Sources: GOC:cjm Also known as: PL scrambling, phospholipid scrambling Relationships: is a type of plasma membrane organization [GO:0007009]; is a type of phospholipid translocation [GO:0045332] Definition: The movement of a population of phospholipid molecules from one leaflet of the plasma membrane bilayer to the opposite leaflet, resulting in loss of lipid asymmetry and surface exposure of phosphatidylserine (PS) and phosphatidylethanolamine (PE). Note: Note that this term describes the trans-bilayer motion of a population of phospholipid molecules, and should not be confused with 'phospholipid translocation ; GO:0045332'.